{
  "term_label": "SUMO ligase activity",
  "term_id": "GO:0061665",
  "gene": "UniProtKB:O75925",
  "gene_name": "E3 SUMO-protein ligase PIAS1",
  "gene_symbol": "PIAS1"
}